{
  "gene_name": "Sphingosine 1-phosphate receptor 1",
  "term_id": "GO:0005737",
  "gene_symbol": "S1PR1",
  "term_label": "cytoplasm",
  "gene": "UniProtKB:P21453"
}